{
  "gene_symbol": "DLX5",
  "gene": "UniProtKB:P56178",
  "gene_name": "Homeobox protein DLX-5",
  "term_id": "GO:0000981",
  "term_label": "DNA-binding transcription factor activity, RNA polymerase II-specific"
}